{
  "gene_name": "DNA excision repair protein ERCC-1",
  "term_id": "GO:0003684",
  "gene": "UniProtKB:P07992",
  "gene_symbol": "ERCC1",
  "term_label": "damaged DNA binding"
}